{
  "gene_name": "Ras-related C3 botulinum toxin substrate 2",
  "term_id": "GO:0007163",
  "gene": "UniProtKB:P15153",
  "term_label": "establishment or maintenance of cell polarity",
  "gene_symbol": "RAC2"
}